{
  "gene": "UniProtKB:A4D1S5",
  "gene_symbol": "RAB19",
  "term_id": "GO:0000045",
  "term_label": "autophagosome assembly",
  "gene_name": "Ras-related protein Rab-19"
}